{
  "gene": "UniProtKB:Q9UJ90",
  "term_label": "potassium ion export across plasma membrane",
  "gene_symbol": "KCNE5",
  "gene_name": "Potassium voltage-gated channel subfamily E regulatory beta subunit 5",
  "term_id": "GO:0097623"
}